{
  "gene_name": "Phosphomevalonate kinase",
  "term_label": "cholesterol biosynthetic process",
  "gene": "UniProtKB:Q15126",
  "term_id": "GO:0006695",
  "gene_symbol": "PMVK"
}